{
  "gene_symbol": "CEP350",
  "gene_name": "Centrosome-associated protein 350",
  "term_id": "UNKNOWN:0003",
  "term_label": "Unknown cellular component",
  "gene": "UniProtKB:Q5VT06"
}